{
  "term_id": "GO:0030317",
  "term_label": "flagellated sperm motility",
  "gene_symbol": "TMEM232",
  "gene_name": "Transmembrane protein 232",
  "gene": "UniProtKB:C9JQI7"
}